{
  "term_id": "UNKNOWN:0003",
  "gene_name": "Immunoglobulin heavy variable 4-31",
  "gene": "UniProtKB:P0DP07",
  "term_label": "Unknown cellular component",
  "gene_symbol": "IGHV4-31"
}